{
  "term_label": "extracellular space",
  "gene_symbol": "SERPINC1",
  "gene": "UniProtKB:P01008",
  "term_id": "GO:0005615",
  "gene_name": "Antithrombin-III"
}